{
  "gene_symbol": "FRZB",
  "term_label": "extracellular space",
  "gene_name": "Secreted frizzled-related protein 3",
  "gene": "UniProtKB:Q92765",
  "term_id": "GO:0005615"
}